pyridine nucleoside catabolic process [GO:0070638] (biological process) Sources: GOC:mah Relationships: is a type of nucleoside catabolic process [GO:0009164]; is a type of GO:0070637; is a type of pyridine-containing compound catabolic process [GO:0072526] Also known as: pyridine nucleoside breakdown, pyridine nucleoside catabolism, pyridine nucleoside degradation Definition: The chemical reactions and pathways resulting in the breakdown of any pyridine nucleoside, a nucleoside in which a pyridine base covalently bonded to a sugar, usually ribose. Subtypes: nicotinamide riboside catabolic process [GO:0006738]